{
  "term_id": "UNKNOWN:0003",
  "gene_name": "Probable inactive 1-aminocyclopropane-1-carboxylate synthase-like protein 2",
  "term_label": "Unknown cellular component",
  "gene_symbol": "ACCSL",
  "gene": "UniProtKB:Q4AC99"
}